peptide lactyltransferase (CoA-dependent) activity [GO:0120300] (molecular function) Also known as: peptide lactyltransferase (CoA dependent) activity, peptide lactyltransferase activity, peptide lactyltransferase activity (CoA-dependent) Subtypes: histone lactyltransferase (CoA-dependent) activity [GO:0120301] References: PMID:31645732 Sources: GOC:sp, RHEA:61996 Definition: Catalysis of the reaction: (L-lysyl-[protein] + lactoyl-CoA = CoA + H+ + N(6)-lactoyl-L-lysyl-[protein]. Relationships: is a type of N-acyltransferase activity [GO:0016410]